{
  "gene_symbol": "USH2A",
  "gene": "UniProtKB:O75445",
  "gene_name": "Usherin",
  "term_label": "Unknown cellular component",
  "term_id": "UNKNOWN:0003"
}